{
  "gene": "UniProtKB:P35504",
  "gene_name": "UDP-glucuronosyltransferase 1A5",
  "term_label": "estrogen metabolic process",
  "gene_symbol": "UGT1A5",
  "term_id": "GO:0008210"
}